{
  "gene_symbol": "PYDC2",
  "gene": "UniProtKB:Q56P42",
  "term_id": "UNKNOWN:0003",
  "term_label": "Unknown cellular component",
  "gene_name": "Pyrin domain-containing protein 2"
}